regulation of myeloid dendritic cell chemotaxis [GO:2000527] (biological process) Definition: Any process that modulates the frequency, rate or extent of myeloid dendritic cell chemotaxis. Subtypes: GO:2000528, GO:2000529 Sources: GOC:obol Relationships: is a type of regulation of dendritic cell chemotaxis [GO:2000508]; regulates myeloid dendritic cell chemotaxis [GO:0002408]